{
  "gene_name": "Bifunctional UDP-N-acetylglucosamine 2-epimerase_N-acetylmannosamine kinase",
  "term_id": "GO:0008761",
  "gene": "UniProtKB:Q9Y223",
  "term_label": "UDP-N-acetylglucosamine 2-epimerase activity",
  "gene_symbol": "GNE"
}